24S-hydroxycholesterol 7-alpha-hydroxylase activity [GO:0033782] (molecular function) References: PMID:10748047, PMID:11013305 Sources: RHEA:46124 Definition: Catalysis of the reaction: (24S)-hydroxycholesterol + O2 + reduced [NADPH-hemoprotein reductase] = (24S)-7alpha-dihydroxycholesterol + H+ + H2O + oxidized [NADPH-hemoprotein reductase]. Also known as: 24-hydroxycholesterol 7alpha-hydroxylase activity, 24-cholest-5-ene-3beta,24-diol,NADPH:oxygen oxidoreductase (7alpha-hydroxylating) activity, 24-hydroxycholesterol 7alpha-monooxygenase activity Relationships: is a type of steroid 7-alpha-hydroxylase activity [GO:0008387]; is a type of oxidoreductase activity, acting on paired donors, with incorporation or reduction of molecular oxygen, reduced flavin or flavoprotein as one donor, and incorporation of one atom of oxygen [GO:0016712]